{
  "term_id": "GO:0005856",
  "gene_name": "Leiomodin-1",
  "gene": "UniProtKB:P29536",
  "gene_symbol": "LMOD1",
  "term_label": "cytoskeleton"
}